{
  "term_id": "GO:0005737",
  "gene": "UniProtKB:Q9UH17",
  "gene_name": "DNA dC-dU-editing enzyme APOBEC-3B",
  "gene_symbol": "APOBEC3B",
  "term_label": "cytoplasm"
}